{
  "term_id": "UNKNOWN:0002",
  "term_label": "Unknown biological process",
  "gene_name": "CD81 antigen",
  "gene": "UniProtKB:P60033",
  "gene_symbol": "CD81"
}